{
  "term_id": "GO:0051156",
  "gene": "UniProtKB:P35557",
  "gene_symbol": "GCK",
  "term_label": "glucose 6-phosphate metabolic process",
  "gene_name": "Hexokinase-4"
}